{
  "gene_name": "Protein pelota homolog",
  "term_id": "UNKNOWN:0001",
  "gene": "UniProtKB:Q9BRX2",
  "gene_symbol": "PELO",
  "term_label": "Unknown molecular function"
}